{
  "term_id": "UNKNOWN:0001",
  "term_label": "Unknown molecular function",
  "gene_name": "Uncharacterized protein C13orf42",
  "gene_symbol": "C13orf42",
  "gene": "UniProtKB:A0A1B0GVH6"
}